{
  "term_label": "RNA polymerase II transcription regulatory region sequence-specific DNA binding",
  "gene_name": "Zinc finger protein 69 homolog B",
  "gene_symbol": "ZFP69B",
  "term_id": "GO:0000977",
  "gene": "UniProtKB:Q9UJL9"
}